intrinsic apoptotic signaling pathway by p53 class mediator [GO:0072332] (biological process) Relationships: is a type of signal transduction by p53 class mediator [GO:0072331]; is a type of GO:0097193 Subtypes: intrinsic apoptotic signaling pathway in response to DNA damage by p53 class mediator [GO:0042771], intrinsic apoptotic signaling pathway in response to osmotic stress by p53 class mediator [GO:1990127] Definition: The series of molecular signals in which an intracellular signal is conveyed to trigger the apoptotic death of a cell. The pathway is induced by the cell cycle regulator phosphoprotein p53, or an equivalent protein, and ends when the execution phase of apoptosis is triggered. Also known as: intrinsic apoptotic signaling pathway by signal transduction by p53 class mediator, signal transduction by p53 class mediator resulting in induction of apoptosis Regulation: regulated by regulation of intrinsic apoptotic signaling pathway by p53 class mediator [GO:1902253]; RO_0002212 by negative regulation of intrinsic apoptotic signaling pathway by p53 class mediator [GO:1902254]; positively regulated by positive regulation of intrinsic apoptotic signaling pathway by p53 class mediator [GO:1902255] Sources: GOC:mah, GOC:mtg_apoptosis